{
  "gene_name": "Cysteine protease ATG4A",
  "term_label": "aggrephagy",
  "gene_symbol": "ATG4A",
  "term_id": "GO:0035973",
  "gene": "UniProtKB:Q8WYN0"
}